{
  "term_id": "GO:0006427",
  "term_label": "histidyl-tRNA aminoacylation",
  "gene_symbol": "HARS2",
  "gene": "UniProtKB:P49590",
  "gene_name": "Histidine--tRNA ligase, mitochondrial"
}